regulation of substrate adhesion-dependent cell spreading [GO:1900024] (biological process) Definition: Any process that modulates the frequency, rate or extent of substrate adhesion-dependent cell spreading. Sources: GOC:TermGenie, GOC:yaf Also known as: regulation of cell spreading during cell substrate adhesion, regulation of substrate adhesion dependent cell spreading Relationships: is a type of regulation of cell-substrate adhesion [GO:0010810]; regulates GO:0034446 Subtypes: negative regulation of substrate adhesion-dependent cell spreading [GO:1900025], GO:1900026